Golgi to vacuole transport [GO:0006896] (biological process) Sources: GOC:ai Definition: The directed movement of substances from the Golgi to the vacuole. Also known as: Golgi to vacuole vesicle-mediated transport Relationships: is a type of post-Golgi vesicle-mediated transport [GO:0006892]; is a type of vacuolar transport [GO:0007034] Subtypes: Golgi to lysosome transport [GO:0090160]